{
  "term_label": "actin filament binding",
  "gene": "UniProtKB:Q9Y281",
  "gene_name": "Cofilin-2",
  "term_id": "GO:0051015",
  "gene_symbol": "CFL2"
}